{
  "term_label": "endosomal transport",
  "term_id": "GO:0016197",
  "gene_name": "Annexin A8",
  "gene": "UniProtKB:P13928",
  "gene_symbol": "ANXA8"
}